{
  "gene_symbol": "CC2D2A",
  "term_id": "GO:1905515",
  "gene": "UniProtKB:Q9P2K1",
  "gene_name": "Coiled-coil and C2 domain-containing protein 2A",
  "term_label": "non-motile cilium assembly"
}